regulation of response to ethanol [GO:1901416] (BP) Sources: GOC:TermGenie, GOC:mengo_curators Relationships: is a type of GO:1901419; regulates GO:0045471 Subtypes: GO:1901417, positive regulation of response to ethanol [GO:1901418] Definition: Any process that modulates the frequency, rate or extent of response to ethanol.